{
  "gene": "UniProtKB:Q6F5E7",
  "term_label": "Unknown molecular function",
  "gene_symbol": "TXNRD3NB",
  "term_id": "UNKNOWN:0001",
  "gene_name": "Putative uncharacterized protein TXNRD3NB"
}